{
  "term_id": "GO:0004714",
  "term_label": "transmembrane receptor protein tyrosine kinase activity",
  "gene": "UniProtKB:P04626",
  "gene_name": "Receptor tyrosine-protein kinase erbB-2",
  "gene_symbol": "ERBB2"
}